{
  "gene": "UniProtKB:O75570",
  "term_label": "Unknown molecular function",
  "gene_name": "Peptide chain release factor 1, mitochondrial",
  "gene_symbol": "MTRF1",
  "term_id": "UNKNOWN:0001"
}